{
  "gene_symbol": "ZNF536",
  "term_id": "GO:0000981",
  "gene": "UniProtKB:O15090",
  "gene_name": "Zinc finger protein 536",
  "term_label": "DNA-binding transcription factor activity, RNA polymerase II-specific"
}